anterior lateral line neuromast deposition [GO:0048902] (biological process) Relationships: is a type of GO:0048885; BFO_0000050 GO:0048901 References: PMID:15832385 Definition: The process in which a migrating neuromast primordium deposits clusters of undifferentiated cells (proneuromasts) along its migratory path in the developing anterior lateral line.